{
  "term_id": "UNKNOWN:0001",
  "gene_name": "PGAP2-interacting protein",
  "gene": "UniProtKB:Q9H720",
  "term_label": "Unknown molecular function",
  "gene_symbol": "CWH43"
}